negative regulation of histamine uptake [GO:0051617] (BP) Relationships: is a type of negative regulation of neurotransmitter uptake [GO:0051581]; is a type of regulation of histamine uptake [GO:0051616]; negatively regulates GO:0051615 Definition: Any process that stops, prevents, or reduces the frequency, rate or extent of the directed movement of histamine into a cell. Also known as: down regulation of histamine uptake, down-regulation of histamine uptake, downregulation of histamine uptake, negative regulation of histamine import Sources: GOC:ai Subtypes: inhibition of histamine uptake [GO:0051619]